{
  "term_id": "GO:0002009",
  "term_label": "morphogenesis of an epithelium",
  "gene": "UniProtKB:Q6A163",
  "gene_name": "Keratin, type I cytoskeletal 39",
  "gene_symbol": "KRT39"
}